leptin receptor binding [GO:1990460] (molecular function) Definition: Binding to a leptin receptor. References: PMID:22405007 Sources: GOC:pm Relationships: is a type of signaling receptor binding [GO:0005102]